transmembrane phosphate ion transport from cytosol to vacuole [GO:1905011] (biological process) Definition: The directed movement of phosphate ions from the cytosol across the vacuolar membrane and into the vacuolar lumen. References: PMID:26554016 Sources: GOC:TermGenie, GO_REF:0000078 Relationships: is a type of GO:0034486; is a type of GO:0035435 Also known as: vacuolar phosphate transport